{
  "gene": "UniProtKB:Q8NEG5",
  "term_label": "Unknown molecular function",
  "term_id": "UNKNOWN:0001",
  "gene_name": "E3 ubiquitin-protein ligase ZSWIM2",
  "gene_symbol": "ZSWIM2"
}